{
  "gene": "UniProtKB:O60333",
  "term_id": "GO:0005737",
  "term_label": "cytoplasm",
  "gene_name": "Kinesin-like protein KIF1B",
  "gene_symbol": "KIF1B"
}